monoterpene biosynthetic process [GO:0043693] (biological process) Definition: The chemical reactions and pathways resulting in the formation of monoterpenes, terpenes with a C10 structure. Relationships: is a type of monoterpene metabolic process [GO:0043692]; is a type of terpene biosynthetic process [GO:0046246] Subtypes: alpha-pinene biosynthetic process [GO:0046248], GO:0046250 Sources: Wikipedia:Monoterpene Also known as: monoterpene biosynthesis